follicle cell of egg chamber development [GO:0030707] (biological process) Relationships: is a type of epithelial cell development [GO:0002064]; is_a developmental process involved in reproduction [GO:0003006]; is part of oogenesis [GO:0048477] Definition: The process that occurs during oogenesis involving the ovarian follicle cells, somatic cells which surround the germ cells of an ovary. An example of this is found in Drosophila melanogaster. References: PMID:10822261 Sources: GOC:mtg_sensu